interleukin-6 receptor complex [GO:0005896] (cellular component) References: PMID:8083235 Also known as: IL-6 receptor complex Relationships: is a type of plasma membrane signaling receptor complex [GO:0098802] Definition: A hexameric protein complex consisting of two molecules each of interleukin-6, interleukin-6 receptor alpha chain, and gp-130.